{
  "gene": "UniProtKB:Q96GX8",
  "term_label": "Unknown molecular function",
  "gene_name": "Uncharacterized protein C16orf74",
  "term_id": "UNKNOWN:0001",
  "gene_symbol": "C16orf74"
}